regulation of double-strand break repair [GO:2000779] (biological process) Subtypes: regulation of double-strand break repair via homologous recombination [GO:0010569], GO:1903776, GO:2000780, positive regulation of double-strand break repair [GO:2000781], regulation of double-strand break repair via nonhomologous end joining [GO:2001032] Definition: Any process that modulates the frequency, rate or extent of double-strand break repair. Sources: GOC:BHF Relationships: is a type of regulation of DNA repair [GO:0006282]; regulates double-strand break repair [GO:0006302]